axon target recognition [GO:0007412] (biological process) Sources: ISBN:0878932437 Definition: The process in which an axon recognizes and binds to a set of cells with which it may form stable connections. Relationships: is a type of GO:0007154; is part of axonogenesis [GO:0007409]